{
  "gene_name": "Neurite extension and migration factor",
  "term_id": "GO:2001223",
  "gene": "UniProtKB:Q5QGS0",
  "gene_symbol": "NEXMIF",
  "term_label": "negative regulation of neuron migration"
}